{
  "term_label": "respiratory chain complex I",
  "gene_symbol": "NDUFB4",
  "gene_name": "NADH dehydrogenase [ubiquinone] 1 beta subcomplex subunit 4",
  "term_id": "GO:0045271",
  "gene": "UniProtKB:O95168"
}